{
  "term_id": "GO:0097320",
  "term_label": "plasma membrane tubulation",
  "gene_symbol": "BIN3",
  "gene_name": "Bridging integrator 3",
  "gene": "UniProtKB:Q9NQY0"
}